nuclear migration [GO:0007097] (biological process) Also known as: establishment of position of nucleus, nuclear movement, nuclear positioning, nucleus migration, nucleus positioning, positioning of nucleus, establishment of cell nucleus localization, establishment of localization of nucleus, establishment of nucleus localisation, establishment of nucleus localization Relationships: is_a intracellular transport [GO:0046907]; is a type of GO:0051647; is a type of GO:0051656 Subtypes: nuclear migration involved in conjugation with mutual genetic exchange [GO:0000745], oocyte nucleus migration involved in oocyte dorsal/ventral axis specification [GO:0007312], embryo sac nuclear migration [GO:0009562], interkinetic nuclear migration [GO:0022027], nuclear migration along microtubule [GO:0030473], nuclear migration along microfilament [GO:0031022], pronuclear migration [GO:0035046], syncytial nuclear migration [GO:0035190], nuclear migration by microtubule mediated pushing forces [GO:0098863], GO:1990974 Definition: The directed movement of the nucleus to a specific location within a cell. Sources: GOC:ai